{
  "term_label": "plasma membrane",
  "gene_name": "Epidermal growth factor receptor kinase substrate 8",
  "gene": "UniProtKB:Q12929",
  "gene_symbol": "EPS8",
  "term_id": "GO:0005886"
}